{
  "term_id": "UNKNOWN:0002",
  "gene_name": "Alpha-protein kinase 2",
  "gene_symbol": "ALPK2",
  "term_label": "Unknown biological process",
  "gene": "UniProtKB:Q86TB3"
}